{
  "term_label": "Unknown biological process",
  "term_id": "UNKNOWN:0002",
  "gene_symbol": "SHISA4",
  "gene_name": "Protein shisa-4",
  "gene": "UniProtKB:Q96DD7"
}